{
  "gene_name": "Cytokine SCM-1 beta",
  "gene_symbol": "XCL2",
  "term_label": "cell chemotaxis",
  "term_id": "GO:0060326",
  "gene": "UniProtKB:Q9UBD3"
}